response to purine-containing compound [GO:0014074] (biological process) Subtypes: response to caffeine [GO:0031000], response to ATP [GO:0033198], response to cAMP [GO:0051591], response to cGMP [GO:0070305], cellular response to purine-containing compound [GO:0071415], GO:1901560, response to reversine [GO:1901596], response to cordycepin [GO:1904309], response to puromycin [GO:1905794] Sources: GOC:ef Definition: Any process that results in a change in state or activity of a cell or an organism (in terms of movement, secretion, enzyme production, gene expression, etc.) as a result of a purine-containing compound stimulus. Relationships: is a type of response to nitrogen compound [GO:1901698] Also known as: response to purine